positive regulation of Golgi vesicle fusion to target membrane [GO:0048215] (biological process) Relationships: is a type of positive regulation of vesicle fusion [GO:0031340]; is a type of regulation of Golgi vesicle fusion to target membrane [GO:0048214]; positively regulates GO:0048210 Also known as: up regulation of Golgi vesicle fusion to target membrane, up-regulation of Golgi vesicle fusion to target membrane, upregulation of Golgi vesicle fusion to target membrane, activation of Golgi vesicle fusion to target membrane, stimulation of Golgi vesicle fusion to target membrane Definition: Any process that activates or increases the frequency, rate or extent of Golgi vesicle fusion to target membrane. References: PMID:10219233 Sources: GOC:jid, ISBN:0716731363